{
  "gene": "UniProtKB:P01880",
  "term_id": "GO:0034987",
  "term_label": "immunoglobulin receptor binding",
  "gene_name": "Immunoglobulin heavy constant delta",
  "gene_symbol": "IGHD"
}